{
  "term_id": "GO:0045747",
  "gene_symbol": "POGLUT1",
  "gene_name": "Protein O-glucosyltransferase 1",
  "term_label": "positive regulation of Notch signaling pathway",
  "gene": "UniProtKB:Q8NBL1"
}